{
  "term_label": "Unknown cellular component",
  "gene_name": "Serine_threonine-protein kinase Nek5",
  "term_id": "UNKNOWN:0003",
  "gene_symbol": "NEK5",
  "gene": "UniProtKB:Q6P3R8"
}